{
  "gene_name": "Long-chain specific acyl-CoA dehydrogenase, mitochondrial",
  "gene": "UniProtKB:P28330",
  "term_id": "GO:0005739",
  "gene_symbol": "ACADL",
  "term_label": "mitochondrion"
}